type 2 immune response [GO:0042092] (biological process) Regulation: RO_0002211 by GO:0002828; negatively regulated by negative regulation of type 2 immune response [GO:0002829]; positively regulated by GO:0002830 Relationships: is a type of GO:0006955 References: PMID:18000958, PMID:18007680, PMID:20065995, PMID:20200518 Sources: GOC:add, ISBN:0781735149 Also known as: T-helper 2 type immune response, Th2 immune response Definition: An immune response which is associated with resistance to extracellular organisms such as helminths and pathological conditions such as allergy, which is orchestrated by the production of particular cytokines, most notably IL-4, IL-5, IL-10, and IL-13, by any of a variety of cell types including T-helper 2 cells, eosinophils, basophils, mast cells, and nuocytes, resulting in enhanced production of certain antibody isotypes and other effects.